{
  "gene": "UniProtKB:Q15942",
  "term_label": "integrin-mediated signaling pathway",
  "gene_name": "Zyxin",
  "gene_symbol": "ZYX",
  "term_id": "GO:0007229"
}